{
  "term_id": "GO:0019221",
  "term_label": "cytokine-mediated signaling pathway",
  "gene": "UniProtKB:P15260",
  "gene_name": "Interferon gamma receptor 1",
  "gene_symbol": "IFNGR1"
}